{
  "term_id": "GO:0005388",
  "gene_name": "Sarcoplasmic_endoplasmic reticulum calcium ATPase 1",
  "gene_symbol": "ATP2A1",
  "term_label": "P-type calcium transporter activity",
  "gene": "UniProtKB:O14983"
}